{
  "term_id": "GO:0030833",
  "gene_symbol": "PFN3",
  "term_label": "regulation of actin filament polymerization",
  "gene_name": "Profilin-3",
  "gene": "UniProtKB:P60673"
}